{
  "gene": "UniProtKB:P10644",
  "gene_symbol": "PRKAR1A",
  "term_label": "cAMP-dependent protein kinase inhibitor activity",
  "gene_name": "cAMP-dependent protein kinase type I-alpha regulatory subunit",
  "term_id": "GO:0004862"
}